{
  "gene_symbol": "CAMK2B",
  "gene_name": "Calcium_calmodulin-dependent protein kinase type II subunit beta",
  "term_label": "regulation of neuronal synaptic plasticity",
  "gene": "UniProtKB:Q13554",
  "term_id": "GO:0048168"
}